{
  "gene_symbol": "PLPBP",
  "gene_name": "Pyridoxal phosphate homeostasis protein",
  "term_label": "pyridoxal phosphate binding",
  "gene": "UniProtKB:O94903",
  "term_id": "GO:0030170"
}